{
  "term_label": "nucleus",
  "gene_symbol": "CENPA",
  "term_id": "GO:0005634",
  "gene_name": "Histone H3-like centromeric protein A",
  "gene": "UniProtKB:P49450"
}